{
  "gene_symbol": "SYT17",
  "term_label": "plasma membrane",
  "term_id": "GO:0005886",
  "gene_name": "Synaptotagmin-17",
  "gene": "UniProtKB:Q9BSW7"
}